{
  "gene_symbol": "POLR3A",
  "gene": "UniProtKB:O14802",
  "gene_name": "DNA-directed RNA polymerase III subunit RPC1",
  "term_label": "tRNA transcription by RNA polymerase III",
  "term_id": "GO:0042797"
}